nuclear pore nuclear basket [GO:0044615] (CC) Definition: A filamentous, cage-like assembly on the nuclear face of the nuclear pore complex (NPC). In S. cerevisiae, Mlp1p and Mlp2p are two major components of the NPC nuclear basket. In vertebrates, Tpr is a major component. References: PMID:18046406, PMID:19524430, PMID:20947011, PMID:22419078 Sources: GOC:dgf Relationships: is a type of nuclear protein-containing complex [GO:0140513]; is part of nuclear pore [GO:0005643]